{
  "term_label": "neuropeptide binding",
  "gene_symbol": "OPRK1",
  "term_id": "GO:0042923",
  "gene": "UniProtKB:P41145",
  "gene_name": "Kappa-type opioid receptor"
}